{
  "term_id": "UNKNOWN:0002",
  "term_label": "Unknown biological process",
  "gene": "UniProtKB:Q8IZ13",
  "gene_symbol": "FAM200C",
  "gene_name": "Protein FAM200C"
}